regulation of photosynthesis, dark reaction [GO:0010110] (biological process) Sources: GOC:sm Subtypes: regulation of reductive pentose-phosphate cycle [GO:0080152] Relationships: is a type of GO:0010109; is a type of regulation of carbohydrate biosynthetic process [GO:0043255]; regulates photosynthesis, dark reaction [GO:0019685] Definition: Any process that modulates the frequency, rate or extent of photosynthesis dark reaction.